{
  "term_id": "GO:0016757",
  "gene_name": "Post-GPI attachment to proteins factor 4",
  "gene_symbol": "PGAP4",
  "term_label": "glycosyltransferase activity",
  "gene": "UniProtKB:Q9BRR3"
}